{
  "gene_name": "Leucine-rich repeat-containing protein 14B",
  "gene_symbol": "LRRC14B",
  "gene": "UniProtKB:A6NHZ5",
  "term_label": "Unknown cellular component",
  "term_id": "UNKNOWN:0003"
}